{
  "gene_symbol": "ZNF833P",
  "gene_name": "Putative zinc finger protein 833",
  "term_label": "regulation of gene expression",
  "gene": "UniProtKB:Q6ZTB9",
  "term_id": "GO:0010468"
}